nucleotide-sugar metabolic process [GO:0009225] (biological process) Sources: ISBN:0198506732 Also known as: nucleotide-sugar metabolism Definition: The cellular chemical reactions and pathways involving nucleotide-sugars, any nucleotide-carbohydrate in which the distal phosphoric residue of a nucleoside 5'-diphosphate is in glycosidic linkage with a monosaccharide or monosaccharide derivative. Relationships: is a type of nucleoside phosphate metabolic process [GO:0006753]; is a type of GO:1901135 Subtypes: UDP-alpha-D-glucose metabolic process [GO:0006011], UDP-N-acetylglucosamine metabolic process [GO:0006047], nucleotide-sugar biosynthetic process [GO:0009226], GO:0019276, GDP-mannose metabolic process [GO:0019673], GO:0033319, UDP-L-arabinose metabolic process [GO:0033356], GDP-L-fucose metabolic process [GO:0046368], GO:0046381, UDP-glucuronate metabolic process [GO:0046398], UDP-D-galactose metabolic process [GO:0052573]